{
  "term_id": "GO:0043161",
  "gene_name": "E3 ubiquitin-protein ligase COP1",
  "term_label": "proteasome-mediated ubiquitin-dependent protein catabolic process",
  "gene_symbol": "COP1",
  "gene": "UniProtKB:Q8NHY2"
}